{
  "gene_symbol": "ZNF506",
  "term_id": "UNKNOWN:0003",
  "gene_name": "Zinc finger protein 506",
  "term_label": "Unknown cellular component",
  "gene": "UniProtKB:Q5JVG8"
}